{
  "term_id": "UNKNOWN:0001",
  "gene": "UniProtKB:Q567V2",
  "gene_name": "Mpv17-like protein 2",
  "term_label": "Unknown molecular function",
  "gene_symbol": "MPV17L2"
}